guanylate cyclase complex, soluble [GO:0008074] (cellular component) Note: See also the molecular function term 'guanylate cyclase activity ; GO:0004383'. Sources: GOC:mah Definition: Complex that possesses guanylate cyclase activity and is not bound to a membrane. Relationships: is_a GO:1902494; is part of cytosol [GO:0005829]